sympathetic ganglion development [GO:0061549] (biological process) Also known as: sympathetic ganglia development Definition: The process whose specific outcome is the progression of a sympathetic ganglion over time, from its formation to the mature structure. Sources: GOC:BHF, GOC:rl Relationships: is a type of ganglion development [GO:0061548]; is part of sympathetic nervous system development [GO:0048485]